{
  "gene": "UniProtKB:Q96N28",
  "gene_symbol": "PRELID3A",
  "term_id": "GO:1990050",
  "term_label": "phosphatidic acid transfer activity",
  "gene_name": "PRELI domain containing protein 3A"
}